{
  "term_id": "GO:0005737",
  "term_label": "cytoplasm",
  "gene_symbol": "GLE1",
  "gene": "UniProtKB:Q53GS7",
  "gene_name": "mRNA export factor GLE1"
}